chordate pharyngeal muscle development [GO:0043282] (biological process) Relationships: is a type of muscle organ development [GO:0007517]; is part of chordate pharynx development [GO:0160093] Sources: GOC:go_curators Definition: The process whose specific outcome is the progression of the pharyngeal muscle over time, from its formation to the mature structure. A pharyngeal muscle is any muscle that forms part of the pharynx.